snoRNP binding [GO:0030519] (molecular function) Sources: GOC:mah Relationships: is a type of ribonucleoprotein complex binding [GO:0043021] Subtypes: box C/D methylation guide snoRNP complex binding [GO:0062064], box H/ACA snoRNP complex binding [GO:0062065] Definition: Binding to a small nucleolar ribonucleoprotein particle.